peptidyl-tyrosine phosphorylation [GO:0018108] (biological process) Definition: The phosphorylation of peptidyl-tyrosine to form peptidyl-O4'-phospho-L-tyrosine. Relationships: is a type of protein phosphorylation [GO:0006468]; is_a GO:0018212 Subtypes: tyrosine phosphorylation of STAT protein [GO:0007260], GO:0038083, GO:0042976 Sources: RESID:AA0039 Regulation: regulated by GO:0050730; RO_0002213 by GO:0050731; RO_0002212 by negative regulation of peptidyl-tyrosine phosphorylation [GO:0050732]